{
  "gene_symbol": "CASR",
  "gene_name": "Extracellular calcium-sensing receptor",
  "term_id": "GO:0005509",
  "term_label": "calcium ion binding",
  "gene": "UniProtKB:P41180"
}